{
  "gene_name": "X-box-binding protein 1",
  "term_id": "UNKNOWN:0002",
  "gene": "UniProtKB:P17861",
  "term_label": "Unknown biological process",
  "gene_symbol": "XBP1"
}